{
  "gene_symbol": "COL10A1",
  "term_label": "extracellular matrix structural constituent conferring tensile strength",
  "term_id": "GO:0030020",
  "gene_name": "Collagen alpha-1(X) chain",
  "gene": "UniProtKB:Q03692"
}